{
  "term_id": "GO:0032729",
  "gene_symbol": "IL18R1",
  "gene_name": "Interleukin-18 receptor 1",
  "term_label": "positive regulation of type II interferon production",
  "gene": "UniProtKB:Q13478"
}